{
  "gene": "UniProtKB:Q96FN4",
  "gene_symbol": "CPNE2",
  "gene_name": "Copine-2",
  "term_id": "GO:0005544",
  "term_label": "calcium-dependent phospholipid binding"
}